{
  "gene": "UniProtKB:P17010",
  "term_id": "GO:0000978",
  "term_label": "RNA polymerase II cis-regulatory region sequence-specific DNA binding",
  "gene_name": "Zinc finger X-chromosomal protein",
  "gene_symbol": "ZFX"
}